membrane to membrane docking [GO:0022614] (biological process) Also known as: membrane-membrane docking Definition: The initial attachment of a membrane to a target membrane, mediated by proteins protruding from the two membranes. Docking requires only that the membranes come close enough for the proteins to interact and adhere. Sources: GOC:isa_complete Relationships: is a type of membrane docking [GO:0022406]